{
  "gene_name": "Pro-epidermal growth factor",
  "gene_symbol": "EGF",
  "gene": "UniProtKB:P01133",
  "term_label": "positive regulation of MAPK cascade",
  "term_id": "GO:0043410"
}